{
  "gene_symbol": "PECAM1",
  "term_label": "transmembrane signaling receptor activity",
  "gene": "UniProtKB:P16284",
  "gene_name": "Platelet endothelial cell adhesion molecule",
  "term_id": "GO:0004888"
}